{
  "gene": "UniProtKB:Q9UNI6",
  "gene_name": "Dual specificity protein phosphatase 12",
  "gene_symbol": "DUSP12",
  "term_id": "UNKNOWN:0002",
  "term_label": "Unknown biological process"
}